{
  "term_id": "GO:0005737",
  "gene": "UniProtKB:Q9UL33",
  "gene_symbol": "TRAPPC2L",
  "term_label": "cytoplasm",
  "gene_name": "Trafficking protein particle complex subunit 2-like protein"
}